{
  "term_label": "protein serine/threonine kinase activity",
  "term_id": "GO:0004674",
  "gene_symbol": "CDKL4",
  "gene_name": "Cyclin-dependent kinase-like 4",
  "gene": "UniProtKB:Q5MAI5"
}